{
  "gene_name": "Hexokinase-1",
  "gene": "UniProtKB:P19367",
  "term_id": "GO:0008865",
  "gene_symbol": "HK1",
  "term_label": "fructokinase activity"
}